{
  "term_id": "GO:0000398",
  "gene": "UniProtKB:O75526",
  "term_label": "mRNA splicing, via spliceosome",
  "gene_name": "RNA-binding motif protein, X-linked-like-2",
  "gene_symbol": "RBMXL2"
}